{
  "gene_name": "ADP-ribosylation factor-like protein 8B",
  "gene_symbol": "ARL8B",
  "gene": "UniProtKB:Q9NVJ2",
  "term_label": "Unknown molecular function",
  "term_id": "UNKNOWN:0001"
}